deoxyhypusine synthase activity [GO:0034038] (molecular function) Note: Note that this term is equivalent to the obsolete molecular function term 'deoxyhypusine synthase activity ; GO:0004171' and corresponds closely to the biological process term 'deoxyhypusine biosynthetic process from spermidine, using deoxyhypusine synthase ; GO:0050983'. Definition: Catalysis of the reaction: [eIF5A-precursor]-lysine + spermidine = [eIF5A-precursor]-deoxyhypusine + propane-1,3-diamine. Four sub-reactions have been identified,in which the intermediates remain tightly associated with the enzyme: spermidine + NAD+ = dehydrospermidine + NADH; dehydrospermidine + [enzyme]-lysine = N-(4-aminobutylidene)-[enzyme]-lysine + propane-1,3-diamine; N-(4-aminobutylidene)-[enzyme]-lysine + [eIF5A-precursor]-lysine = N-(4-aminobutylidene)-[eIF5A-precursor]-lysine + [enzyme]-lysine; N-(4-aminobutylidene)-[eIF5A-precursor]-lysine + NADH + H+ = [eIF5A-precursor]-deoxyhypusine + NAD+. Also known as: (4-aminobutyl)lysine synthase, spermidine dehydrogenase, eIF-5A-deoxyhypusine synthase activity Relationships: is a type of GO:0016765 Sources: GOC:pde, RHEA:33299